{
  "term_label": "Unknown biological process",
  "gene": "UniProtKB:Q8NCQ2",
  "gene_name": "Uncharacterized protein CSNK1G2-AS1",
  "gene_symbol": "CSNK1G2-AS1",
  "term_id": "UNKNOWN:0002"
}